{
  "gene_symbol": "PRSS51",
  "gene": "UniProtKB:A0A1B0GVH4",
  "gene_name": "Serine protease-like protein 51",
  "term_id": "GO:0005886",
  "term_label": "plasma membrane"
}